endoribonuclease activity, cleaving siRNA-paired mRNA [GO:0070551] (molecular function) Definition: Catalysis of the endonucleolytic cleavage of the mRNA in a double-stranded RNA molecule formed by the base pairing of an mRNA with an siRNA, yielding 5'-phosphomonoesters. References: PMID:15105377 Sources: GOC:mah Also known as: argonaute endoribonuclease activity Relationships: is a type of RNA endonuclease activity producing 5'-phosphomonoesters, hydrolytic mechanism [GO:0016891]